{
  "gene": "UniProtKB:O75400",
  "term_id": "GO:0071004",
  "gene_symbol": "PRPF40A",
  "term_label": "U2-type prespliceosome",
  "gene_name": "Pre-mRNA-processing factor 40 homolog A"
}